{
  "term_id": "UNKNOWN:0001",
  "gene_name": "Small integral membrane protein 5",
  "gene_symbol": "SMIM5",
  "gene": "UniProtKB:Q71RC9",
  "term_label": "Unknown molecular function"
}